{
  "term_id": "GO:0035036",
  "gene_symbol": "FOLR1",
  "gene": "UniProtKB:P15328",
  "gene_name": "Folate receptor alpha",
  "term_label": "sperm-egg recognition"
}